DNA strand elongation involved in nuclear cell cycle DNA replication [GO:1902319] (biological process) Definition: Any DNA strand elongation that is involved in nuclear cell cycle DNA replication. Sources: GOC:TermGenie, GOC:mtg_cell_cycle Also known as: DNA strand elongation involved in DNA replication involved in S phase, DNA strand elongation involved in DNA replication involved in S-phase, DNA strand elongation involved in DNA replication during S phase Relationships: is a type of GO:1902296; is part of nuclear DNA replication [GO:0033260] Subtypes: DNA strand elongation involved in premeiotic DNA replication [GO:1902982], DNA strand elongation involved in mitotic DNA replication [GO:1902983]